semaphorin-plexin signaling pathway involved in outflow tract morphogenesis [GO:0071527] (biological process) References: PMID:15239959 Sources: GOC:BHF, GOC:mah, GOC:vk Regulation: positively regulated by positive regulation of semaphorin-plexin signaling pathway involved in outflow tract morphogenesis [GO:2000764] Definition: The series of molecular signals generated as a consequence of a semaphorin receptor (composed of a plexin and a neurophilin) binding to a semaphorin ligand that contributes to outflow tract morphogenesis. Also known as: semaphorin-plexin signalling pathway involved in outflow tract morphogenesis Relationships: is_a cell surface receptor signaling pathway involved in heart development [GO:0061311]; is a type of semaphorin-plexin signaling pathway [GO:0071526]; is part of GO:0003151